{
  "gene": "UniProtKB:A0A087WXM9",
  "term_label": "male meiosis chromosome segregation",
  "term_id": "GO:0007060",
  "gene_name": "Meiosis-specific kinetochore protein",
  "gene_symbol": "MEIKIN"
}